striated muscle contraction [GO:0006941] (BP) Also known as: sarcomeric muscle contraction Relationships: is a type of muscle contraction [GO:0006936] Regulation: regulated by GO:0006942; negatively regulated by negative regulation of striated muscle contraction [GO:0045988]; positively regulated by GO:0045989 Subtypes: skeletal muscle contraction [GO:0003009], cardiac muscle contraction [GO:0060048], striated muscle contraction involved in embryonic body morphogenesis [GO:0061199] Sources: GOC:jl, GOC:mtg_muscle, ISBN:0198506732 Definition: A process in which force is generated within striated muscle tissue, resulting in the shortening of the muscle. Force generation involves a chemo-mechanical energy conversion step that is carried out by the actin/myosin complex activity, which generates force through ATP hydrolysis. Striated muscle is a type of muscle in which the repeating units (sarcomeres) of the contractile myofibrils are arranged in registry throughout the cell, resulting in transverse or oblique striations observable at the level of the light microscope.